{
  "term_id": "GO:0045047",
  "gene_name": "AN1-type zinc finger protein 2B",
  "gene": "UniProtKB:Q8WV99",
  "gene_symbol": "ZFAND2B",
  "term_label": "protein targeting to ER"
}